{
  "gene_symbol": "RAPGEF4",
  "term_label": "guanyl-nucleotide exchange factor activity",
  "term_id": "GO:0005085",
  "gene": "UniProtKB:Q8WZA2",
  "gene_name": "Rap guanine nucleotide exchange factor 4"
}